{
  "term_id": "GO:0005739",
  "term_label": "mitochondrion",
  "gene_symbol": "SLC25A52",
  "gene": "UniProtKB:Q3SY17",
  "gene_name": "Mitochondrial nicotinamide adenine dinucleotide transporter SLC25A52"
}